{
  "term_id": "GO:2000191",
  "term_label": "regulation of fatty acid transport",
  "gene_symbol": "REPIN1",
  "gene_name": "Replication initiator 1",
  "gene": "UniProtKB:Q9BWE0"
}